{
  "gene_symbol": "AWAT2",
  "gene": "UniProtKB:Q6E213",
  "gene_name": "Acyl-CoA wax alcohol acyltransferase 2",
  "term_id": "GO:0006629",
  "term_label": "lipid metabolic process"
}